regulation of amine catabolic process [GO:0033241] (biological process) Subtypes: negative regulation of amine catabolic process [GO:0033242], positive regulation of amine catabolic process [GO:0033243], GO:1900081 Relationships: is a type of regulation of catabolic process [GO:0009894]; is a type of GO:0033238; regulates amine catabolic process [GO:0009310] Also known as: regulation of amine breakdown, regulation of amine catabolism, regulation of amine degradation, regulation of cellular amine catabolic process Definition: Any process that modulates the frequency, rate or extent of the chemical reactions and pathways leading to the breakdown of amines. Sources: GOC:mah